{
  "gene_name": "Ectonucleoside triphosphate diphosphohydrolase 1",
  "term_id": "GO:0005886",
  "term_label": "plasma membrane",
  "gene": "UniProtKB:P49961",
  "gene_symbol": "ENTPD1"
}